{
  "gene_symbol": "ANKK1",
  "gene_name": "Ankyrin repeat and protein kinase domain-containing protein 1",
  "gene": "UniProtKB:Q8NFD2",
  "term_label": "Unknown molecular function",
  "term_id": "UNKNOWN:0001"
}